{
  "gene_name": "Leukemia-associated protein 7",
  "term_label": "Unknown biological process",
  "term_id": "UNKNOWN:0002",
  "gene_symbol": "DLEU7",
  "gene": "UniProtKB:Q6UYE1"
}